{
  "term_id": "GO:0031023",
  "gene": "UniProtKB:Q99871",
  "gene_symbol": "HAUS7",
  "term_label": "microtubule organizing center organization",
  "gene_name": "HAUS augmin-like complex subunit 7"
}